endocytosed synaptic vesicle to endosome fusion [GO:0099593] (biological process) Relationships: is a type of synaptic vesicle to endosome fusion [GO:0016189]; is part of synaptic vesicle recycling via endosome [GO:0036466] Definition: Fusion of an endocytosed synaptic vesicle with an endosome. Sources: GOC:dos